{
  "term_label": "modulation of chemical synaptic transmission",
  "gene_name": "Glutamate receptor ionotropic, NMDA 3B",
  "gene_symbol": "GRIN3B",
  "gene": "UniProtKB:O60391",
  "term_id": "GO:0050804"
}